{
  "term_label": "Unknown cellular component",
  "gene_name": "Immunoglobulin lambda joining 2 (Fragment)",
  "term_id": "UNKNOWN:0003",
  "gene_symbol": "IGLJ2",
  "gene": "UniProtKB:A0A0A0MT82"
}